{
  "gene_symbol": "A8MZ25",
  "gene_name": "Putative uncharacterized protein FLJ38767",
  "term_label": "Unknown cellular component",
  "gene": "UniProtKB:A8MZ25",
  "term_id": "UNKNOWN:0003"
}